negative regulation of septation initiation signaling [GO:0031030] (biological process) Definition: Any process that stops, prevents, or reduces the frequency, rate or extent of septation initiation signaling. Sources: GOC:mah Also known as: down regulation of septation initiation signaling, down-regulation of septation initiation signaling, downregulation of septation initiation signaling, negative regulation of septation initiation network, negative regulation of septation initiation signalling, inhibition of septation initiation signaling, negative regulation of septation initiation signaling cascade Relationships: is a type of GO:0010974; is a type of GO:0031029; is a type of negative regulation of small GTPase mediated signal transduction [GO:0051058]; negatively regulates septation initiation signaling [GO:0031028]